monocarboxylic acid catabolic process [GO:0072329] (biological process) Definition: The chemical reactions and pathways resulting in the breakdown of monocarboxylic acids, any organic acid containing one carboxyl (-COOH) group. Sources: GOC:mah Relationships: is a type of monocarboxylic acid metabolic process [GO:0032787]; is a type of carboxylic acid catabolic process [GO:0046395] Subtypes: glucuronate catabolic process [GO:0006064], fatty acid catabolic process [GO:0009062], glyoxylate catabolic process [GO:0009436], phenylacetate catabolic process [GO:0010124], pantothenate catabolic process [GO:0015941], 3-phenylpropionate catabolic process [GO:0019380], gallate catabolic process [GO:0019396], mandelate catabolic process [GO:0019596], (R)-4-hydroxymandelate catabolic process [GO:0019599], 3-hydroxyphenylacetate catabolic process [GO:0019610], GO:0019612, 3,4-dihydroxybenzoate catabolic process [GO:0019619], 3-(3-hydroxy)phenylpropionate catabolic process [GO:0019622], quinate catabolic process [GO:0019631], shikimate catabolic process [GO:0019633], mixed acid fermentation [GO:0019664], bile acid catabolic process [GO:0030573], GO:0034653, formate catabolic process [GO:0042183], penicillin catabolic process [GO:0042317], biotin catabolic process [GO:0042367], ectoine catabolic process [GO:0042400], indoleacetic acid catabolic process [GO:0042437], pyruvate catabolic process [GO:0042867], anthranilate catabolic process [GO:0043421], benzoate catabolic process [GO:0043639], GO:0045733, aldonic acid catabolic process [GO:0046176], 2,4,5-trichlorophenoxyacetic acid catabolic process [GO:0046228], salicylic acid catabolic process [GO:0046244], GO:0046276, cinnamic acid catabolic process [GO:0046281], GO:0046296, 2,4-dichlorobenzoate catabolic process [GO:0046298], 2,4-dichlorophenoxyacetic acid catabolic process [GO:0046300], abscisic acid catabolic process [GO:0046345], GO:0046397, 1,6-anhydro-N-acetyl-beta-muramic acid catabolic process [GO:0097175], o-orsellinic acid catabolic process [GO:1900583], ochratoxin A catabolic process [GO:1900817], 4-hydroxyphenylacetate catabolic process [GO:1901023], ferulate catabolic process [GO:1901067], 2-dehydro-3-deoxy-D-gluconic acid catabolic process [GO:1901273], (R)-mevalonic acid catabolic process [GO:1901736], pentalenolactone catabolic process [GO:1901779], p-cumate catabolic process [GO:1901782], GO:1901791, 3-(3-hydroxyphenyl)propanoate catabolic process [GO:1901794], GO:1901848, homogentisate catabolic process [GO:1902000], GO:1902085, glycyrrhetinate catabolic process [GO:1902385], lactate catabolic process [GO:1903457]